ectoine biosynthetic process [GO:0019491] (BP) Also known as: ectoine anabolism, ectoine biosynthesis, ectoine formation, ectoine synthesis Definition: The chemical reactions and pathways resulting in the formation of ectoine (1,4,5,6-tetrahydro-2-methyl-4-pyrimidinecarboxylic acid), a tetrahydropyrimidine commonly synthesized by halophilic bacteria. Relationships: is_a monocarboxylic acid biosynthetic process [GO:0072330] References: PMID:11823218 Sources: GOC:jl